{
  "term_id": "GO:0004143",
  "gene_name": "Diacylglycerol kinase theta",
  "gene_symbol": "DGKQ",
  "term_label": "ATP-dependent diacylglycerol kinase activity",
  "gene": "UniProtKB:P52824"
}